2-dehydro-3-deoxygalactonokinase activity [GO:0008671] (molecular function) Definition: Catalysis of the reaction: 2-dehydro-3-deoxy-D-galactonate + ATP = 6-phospho-2-dehydro-3-deoxy-D-galactonate + ADP + 2 H+. Also known as: 2-keto-3-deoxy-galactonokinase activity, 2-keto-3-deoxygalactonate kinase (phosphorylating), 2-keto-3-deoxygalactonokinase activity, 2-oxo-3-deoxygalactonate kinase activity, ATP:2-dehydro-3-deoxy-D-galactonate 6-phosphotransferase activity Relationships: is a type of phosphotransferase activity, alcohol group as acceptor [GO:0016773]; is a type of carbohydrate kinase activity [GO:0019200] Sources: EC:2.7.1.58, RHEA:16525